{
  "term_id": "GO:0005884",
  "gene": "UniProtKB:P13797",
  "gene_symbol": "PLS3",
  "term_label": "actin filament",
  "gene_name": "Plastin-3"
}